spheroidene monooxygenase activity [GO:0043823] (molecular function) References: PMID:16086104, PMID:16158287 Relationships: is a type of oxidoreductase activity, acting on paired donors, with incorporation or reduction of molecular oxygen, reduced iron-sulfur protein as one donor, and incorporation of one atom of oxygen [GO:0016713] Definition: Catalysis of the reaction: spheroidene + O2 = spheroidenone + H2O.